{
  "gene": "UniProtKB:O43524",
  "gene_symbol": "FOXO3",
  "gene_name": "Forkhead box protein O3",
  "term_id": "GO:0005759",
  "term_label": "mitochondrial matrix"
}